{
  "gene_name": "Ankycorbin",
  "gene": "UniProtKB:Q9P0K7",
  "term_label": "Unknown cellular component",
  "gene_symbol": "RAI14",
  "term_id": "UNKNOWN:0003"
}